{
  "gene_name": "Probable serine carboxypeptidase CPVL",
  "term_id": "GO:0004185",
  "gene_symbol": "CPVL",
  "gene": "UniProtKB:Q9H3G5",
  "term_label": "serine-type carboxypeptidase activity"
}